{
  "term_label": "filopodium assembly",
  "gene_name": "FYVE, RhoGEF and PH domain-containing protein 4",
  "gene": "UniProtKB:Q96M96",
  "term_id": "GO:0046847",
  "gene_symbol": "FGD4"
}